{
  "gene": "UniProtKB:Q9Y6M1",
  "term_id": "GO:0005737",
  "gene_name": "Insulin-like growth factor 2 mRNA-binding protein 2",
  "gene_symbol": "IGF2BP2",
  "term_label": "cytoplasm"
}